{
  "gene_name": "Heat shock 70 kDa protein 12A",
  "gene": "UniProtKB:O43301",
  "term_label": "Unknown biological process",
  "gene_symbol": "HSPA12A",
  "term_id": "UNKNOWN:0002"
}